{
  "gene_symbol": "TSPY1",
  "term_id": "GO:0000785",
  "gene": "UniProtKB:Q01534",
  "term_label": "chromatin",
  "gene_name": "Testis-specific Y-encoded protein 1"
}